{
  "term_id": "GO:0007399",
  "term_label": "nervous system development",
  "gene_name": "Activin receptor type-1C",
  "gene": "UniProtKB:Q8NER5",
  "gene_symbol": "ACVR1C"
}